{
  "term_label": "Unknown molecular function",
  "term_id": "UNKNOWN:0001",
  "gene_name": "Putative uncharacterized protein FER1L6-AS1",
  "gene_symbol": "FER1L6-AS1",
  "gene": "UniProtKB:Q8NA97"
}